{
  "gene_symbol": "RPTOR",
  "gene_name": "Regulatory-associated protein of mTOR",
  "gene": "UniProtKB:Q8N122",
  "term_id": "GO:0005737",
  "term_label": "cytoplasm"
}